{
  "gene": "UniProtKB:P59533",
  "gene_name": "Taste receptor type 2 member 38",
  "gene_symbol": "TAS2R38",
  "term_id": "GO:0033038",
  "term_label": "bitter taste receptor activity"
}